L-phenylalanine conjugated cholate hydrolase activity [GO:7770006] (molecular function) Definition: Catalysis of the reaction: cholate + L-phenylalanine = L-phenylalanocholate + H2O. References: PMID:38326608 Sources: RHEA:79123 Relationships: is a type of amino acid conjugated cholate hydrolase activity [GO:7770003]